uropod organization [GO:0032796] (biological process) References: PMID:12714569, PMID:12787750 Sources: GOC:add, ISBN:0781735149 Subtypes: uropod assembly [GO:0034460], uropod retraction [GO:0034461] Relationships: is a type of plasma membrane bounded cell projection organization [GO:0120036] Definition: A process that is carried out at the cellular level which results in the assembly, arrangement of constituent parts, or disassembly of a uropod, a rigid membrane projection with related cytoskeletal components at the trailing edge of a lymphocyte or other cell in the process of migrating or being activated. Also known as: uropod organisation, uropod organization and biogenesis